transsulfuration [GO:0019346] (biological process) Also known as: transsulphuration, homocysteine-cysteine interconversion Relationships: is a type of cysteine metabolic process [GO:0006534]; is_a homoserine metabolic process [GO:0009092]; is a type of homocysteine metabolic process [GO:0050667] Definition: The interconversion of homocysteine and cysteine via cystathionine. In contrast with enteric bacteria and mammals, Saccharomyces cerevisiae has two transsulfuration pathways employing two separate sets of enzymes. Sources: MetaCyc:PWY-801